{
  "term_id": "UNKNOWN:0003",
  "gene": "UniProtKB:Q9NUM3",
  "gene_name": "Zinc transporter ZIP9",
  "term_label": "Unknown cellular component",
  "gene_symbol": "SLC39A9"
}